cell fate commitment [GO:0045165] (biological process) Definition: The cellular developmental process by which a cell establishes the intrinsic character of a cell or tissue region irreversibly committing it to a particular fate. Sources: ISBN:0716731185 Note: Note that this term was 'cell fate determination' but the term name was changed to better match its existing definition and the child term 'cell fate determination; GO:0001709' was also created. Relationships: is a type of cellular developmental process [GO:0048869]; is part of GO:0030154 Subtypes: inner cell mass cell fate commitment [GO:0001827], trophectodermal cell fate commitment [GO:0001830], osteoblast fate commitment [GO:0002051], B cell lineage commitment [GO:0002326], T cell lineage commitment [GO:0002360], pro-T cell lineage commitment [GO:0002680], determination of imaginal disc primordium [GO:0007445], GO:0010377, GO:0010654, GO:0014017, mesenchymal cell fate commitment [GO:0014030], skeletal muscle satellite cell commitment [GO:0014813], glial cell fate commitment [GO:0021781], GO:0021887, GO:0035854, compound eye cone cell fate commitment [GO:0042676], GO:0042693, oocyte fate commitment [GO:0048600], GO:0048625, neuron fate commitment [GO:0048663], stem cell fate commitment [GO:0048865], GO:0055059, cell fate commitment involved in pattern specification [GO:0060581], GO:0060795, cardiac cell fate commitment [GO:0060911], lens fiber cell fate commitment [GO:0070308], DCT cell fate commitment [GO:0072146], epithelial cell fate commitment [GO:0072148], juxtaglomerulus cell fate commitment [GO:0072150], mesangial cell fate commitment [GO:0072151], renal interstitial fibroblast fate commitment [GO:0072153], proximal convoluted tubule segment 1 cell fate commitment [GO:0072154], GO:0072325, GO:0090106, seed trichome initiation [GO:0090377] Regulation: regulated by regulation of cell fate commitment [GO:0010453]; negatively regulated by negative regulation of cell fate commitment [GO:0010454]; RO_0002213 by positive regulation of cell fate commitment [GO:0010455]